{
  "term_label": "regulation of DNA-templated transcription",
  "term_id": "GO:0006355",
  "gene_name": "Pre-B-cell leukemia transcription factor-interacting protein 1",
  "gene": "UniProtKB:Q96AQ6",
  "gene_symbol": "PBXIP1"
}